{
  "gene_symbol": "MFGE8",
  "term_id": "GO:0005615",
  "gene": "UniProtKB:Q08431",
  "gene_name": "Lactadherin",
  "term_label": "extracellular space"
}